negative regulation of mitotic nuclear envelope disassembly [GO:1905558] (biological process) Definition: Any process that stops, prevents or reduces the frequency, rate or extent of mitotic nuclear envelope disassembly. Relationships: is a type of negative regulation of cell cycle process [GO:0010948]; is a type of negative regulation of cellular component organization [GO:0051129]; is_a GO:1905557; negatively regulates mitotic nuclear membrane disassembly [GO:0007077] Also known as: down regulation of mitotic nuclear envelope breakdown, down regulation of mitotic nuclear envelope catabolism, down regulation of mitotic nuclear envelope degradation, down regulation of mitotic nuclear envelope disassembly, down-regulation of mitotic nuclear envelope breakdown, down-regulation of mitotic nuclear envelope catabolism, down-regulation of mitotic nuclear envelope degradation, down-regulation of mitotic nuclear envelope disassembly, downregulation of mitotic nuclear envelope breakdown, downregulation of mitotic nuclear envelope catabolism, downregulation of mitotic nuclear envelope degradation, downregulation of mitotic nuclear envelope disassembly, negative regulation of mitotic nuclear envelope breakdown, negative regulation of mitotic nuclear envelope catabolism, negative regulation of mitotic nuclear envelope degradation, inhibition of mitotic nuclear envelope breakdown, inhibition of mitotic nuclear envelope catabolism, inhibition of mitotic nuclear envelope degradation, inhibition of mitotic nuclear envelope disassembly References: PMID:18765790 Sources: GOC:TermGenie, GO_REF:0000058